tyrosine-arginine ligase activity [GO:0050367] (molecular function) Also known as: L-tyrosine:L-arginine ligase (AMP-forming), kyotorphin synthase activity, kyotorphin synthetase activity, kyotorphin-synthesizing enzyme activity, tyrosyl-arginine synthase activity Relationships: is_a GO:0016881 Sources: EC:6.3.2.24, RHEA:15345 Definition: Catalysis of the reaction: L-arginine + L-tyrosine + ATP = L-tyrosyl-L-arginine + AMP + diphosphate + 2 H+.